protein-L-histidine N-pros-methyltransferase activity [GO:0106370] (molecular function) Definition: Catalysis of the reaction: L-histidyl-[protein] + S-adenosyl-L-methionine = N(pros)-methyl-L-histidyl-[protein] + S-adenosyl-L-homocysteine. Relationships: is a type of N-methyltransferase activity [GO:0008170]; is a type of GO:0008276; is a type of S-adenosylmethionine-dependent methyltransferase activity [GO:0008757] References: PMID:33563959 Sources: RHEA:67076